retrograde transport, plasma membrane to Golgi [GO:0035526] (BP) Definition: The directed movement of substances from the plasma membrane back to the trans-Golgi network, mediated by vesicles. References: PMID:17488291 Sources: GOC:lb Relationships: is_a vesicle-mediated transport [GO:0016192]